negative regulation of leukocyte activation [GO:0002695] (biological process) Definition: Any process that stops, prevents, or reduces the frequency, rate, or extent of leukocyte activation. Sources: GOC:add Also known as: down regulation of leukocyte activation, down-regulation of leukocyte activation, downregulation of leukocyte activation, negative regulation of immune cell activation, negative regulation of leucocyte activation, inhibition of leukocyte activation Relationships: is a type of negative regulation of immune system process [GO:0002683]; is a type of regulation of leukocyte activation [GO:0002694]; is a type of GO:0050866; negatively regulates leukocyte activation [GO:0045321] Subtypes: negative regulation of myeloid dendritic cell activation [GO:0030886], negative regulation of mast cell activation [GO:0033004], negative regulation of macrophage activation [GO:0043031], negative regulation of lymphocyte activation [GO:0051250], GO:0150102, negative regulation of neutrophil activation [GO:1902564], negative regulation of eosinophil activation [GO:1902567]